{
  "term_id": "GO:0005886",
  "term_label": "plasma membrane",
  "gene": "UniProtKB:Q9NR61",
  "gene_symbol": "DLL4",
  "gene_name": "Delta-like protein 4"
}